{
  "term_label": "cell differentiation",
  "gene_name": "Eyes absent homolog 4",
  "term_id": "GO:0030154",
  "gene": "UniProtKB:O95677",
  "gene_symbol": "EYA4"
}